{
  "gene_symbol": "ZNF333",
  "term_label": "RNA polymerase II cis-regulatory region sequence-specific DNA binding",
  "gene_name": "Zinc finger protein 333",
  "gene": "UniProtKB:Q96JL9",
  "term_id": "GO:0000978"
}